{
  "term_label": "plasma membrane",
  "term_id": "GO:0005886",
  "gene": "UniProtKB:P98164",
  "gene_symbol": "LRP2",
  "gene_name": "Low-density lipoprotein receptor-related protein 2"
}